{
  "gene": "UniProtKB:Q9H213",
  "gene_name": "Melanoma-associated antigen H1",
  "term_id": "GO:0005634",
  "gene_symbol": "MAGEH1",
  "term_label": "nucleus"
}